{
  "gene_name": "Putative uncharacterized protein ENSP00000382790",
  "gene": "UniProtKB:A8MVM7",
  "gene_symbol": "A8MVM7",
  "term_id": "UNKNOWN:0001",
  "term_label": "Unknown molecular function"
}